signal peptidase activity [GO:0009003] (MF) Relationships: is a type of endopeptidase activity [GO:0004175] Definition: An endopeptidase that cleaves a hydrophobic, N-terminal signal or leader sequences from mitochondrial, secreted and periplasmic proteins. Sources: GOC:vw Note: Note that this term was reinstated from obsolete.